{
  "term_id": "GO:0000981",
  "gene_name": "Myocyte-specific enhancer factor 2B",
  "term_label": "DNA-binding transcription factor activity, RNA polymerase II-specific",
  "gene": "UniProtKB:Q02080",
  "gene_symbol": "MEF2B"
}